{
  "term_id": "GO:0005634",
  "gene": "UniProtKB:Q9P287",
  "gene_symbol": "BCCIP",
  "gene_name": "BRCA2 and CDKN1A-interacting protein",
  "term_label": "nucleus"
}